{
  "gene_name": "Zinc finger protein 705D",
  "gene": "UniProtKB:P0CH99",
  "gene_symbol": "ZNF705D",
  "term_id": "GO:0005634",
  "term_label": "nucleus"
}